spermatoproteasome complex [GO:1990111] (cellular component) Definition: A proteasome specifically found in mammalian testis. Contains the proteasome activator PA200 in the regulatory particle, and beta1i, beta2i, beta5i and/or alpha4s in the core (20S) subunit. Beta1i, beta2i and beta5i are inducible catalytic subunits, closely related to beta1, beta2 and beta5. Alpha4s is a sperm-specific 20S subunit, but unlike other alternative 20S subunits alpha4s lies in the outer alpha-ring and lacks catalytic activity. References: PMID:23706739 Sources: GOC:sp Relationships: is a type of proteasome complex [GO:0000502]